chemokine-mediated signaling pathway [GO:0070098] (biological process) Sources: GOC:mah, GOC:signaling Relationships: is a type of G protein-coupled receptor signaling pathway [GO:0007186]; is a type of GO:0019221; is part of cellular response to chemokine [GO:1990869] Also known as: chemokine-mediated signalling pathway Definition: The series of molecular signals initiated by a chemokine binding to its receptor on the surface of a target cell, and ending with the regulation of a downstream cellular process, e.g. transcription. Subtypes: GO:0035689, chemokine (C-C motif) ligand 19 signaling pathway [GO:0038115], chemokine (C-C motif) ligand 21 signaling pathway [GO:0038116], GO:0038118, GO:0038146, chemokine (C-C motif) ligand 2 signaling pathway [GO:0038148], C-C chemokine receptor CCR2 signaling pathway [GO:0038150], C-C chemokine receptor CCR4 signaling pathway [GO:0038152], C-X-C chemokine receptor CXCR4 signaling pathway [GO:0038159], thrombopoietin-mediated signaling pathway [GO:0038163] Regulation: regulated by regulation of chemokine-mediated signaling pathway [GO:0070099]; negatively regulated by negative regulation of chemokine-mediated signaling pathway [GO:0070100]; positively regulated by positive regulation of chemokine-mediated signaling pathway [GO:0070101]